dolichyl-phosphate-mannose-protein mannosyltransferase Pmt5p-Pmt2p dimer complex [GO:0097584] (cellular component) Definition: A protein dimer complex that possesses dolichyl-phosphate-mannose-protein mannosyltransferase activity and, in S. cerevisiae, is composed of Pmt5p-Pmt2p. Also known as: Pmt5p-Pmt2p complex References: PMID:12551906 Sources: GOC:jd Relationships: is a type of dolichyl-phosphate-mannose-protein mannosyltransferase complex [GO:0031502]